{
  "term_label": "antigen processing and presentation of peptide antigen via MHC class II",
  "gene_name": "E3 ubiquitin-protein ligase MARCHF8",
  "gene_symbol": "MARCHF8",
  "term_id": "GO:0002495",
  "gene": "UniProtKB:Q5T0T0"
}